{
  "gene_name": "Forkhead box protein G1",
  "gene_symbol": "FOXG1",
  "term_id": "GO:0006357",
  "term_label": "regulation of transcription by RNA polymerase II",
  "gene": "UniProtKB:P55316"
}